positive regulation of cellular response to hepatocyte growth factor stimulus [GO:2001114] (biological process) Relationships: is a type of positive regulation of response to stimulus [GO:0048584]; is a type of regulation of cellular response to hepatocyte growth factor stimulus [GO:2001112]; positively regulates cellular response to hepatocyte growth factor stimulus [GO:0035729] Sources: GOC:obol Also known as: positive regulation of cellular response to HGF stimulus Definition: Any process that activates or increases the frequency, rate or extent of cellular response to hepatocyte growth factor stimulus.